{
  "gene_symbol": "ZNF418",
  "term_id": "GO:0006357",
  "gene_name": "Zinc finger protein 418",
  "gene": "UniProtKB:Q8TF45",
  "term_label": "regulation of transcription by RNA polymerase II"
}